pentachlorophenol catabolic process [GO:0019338] (biological process) Relationships: is a type of phenol-containing compound catabolic process [GO:0019336]; is a type of benzene-containing compound metabolic process [GO:0042537]; is a type of organohalogen metabolic process [GO:0090345] Sources: GOC:go_curators Also known as: pentachlorophenol breakdown, pentachlorophenol catabolism, pentachlorophenol degradation Definition: The chemical reactions and pathways resulting in the breakdown of pentachlorophenol, a chlorinated insecticide and fungicide used primarily to protect timber from fungal rot and wood boring insects. Pentachlorophenol is significantly toxic to mammals, plants, and many microorganisms.